{
  "term_id": "GO:0005737",
  "gene": "UniProtKB:Q9NWD9",
  "gene_symbol": "BEX4",
  "term_label": "cytoplasm",
  "gene_name": "Protein BEX4"
}